{
  "term_label": "kinetochore",
  "term_id": "GO:0000776",
  "gene_symbol": "CENPW",
  "gene": "UniProtKB:Q5EE01",
  "gene_name": "Centromere protein W"
}